dipeptide transmembrane transport from lysosomal lumen to cytosol [GO:0141204] (BP) Definition: The directed movement of dipeptide from the lysosomal lumen across the lysosomal membrane and into the cytosol. References: PMID:38507452 Relationships: is a type of peptide transport [GO:0015833]; is_a transmembrane transport from lysosomal lumen to cytosol [GO:0170063] Also known as: dipeptide export from lysosomal lumen, dipeptide export from lysosome, transmembrane dipeptide transport from lysosomal lumen to cytosol